N-carbamoylsarcosine amidase activity [GO:0050127] (molecular function) Definition: Catalysis of the reaction: N-carbamoylsarcosine + H2O + 2 H+ = CO2 + NH4 + sarcosine. Sources: EC:3.5.1.59, RHEA:20057 Also known as: CSHase activity, N-carbamoylsarcosine amidohydrolase activity, carbamoylsarcosine amidase activity Relationships: is a type of hydrolase activity, acting on carbon-nitrogen (but not peptide) bonds, in linear amides [GO:0016811]